female germline ring canal [GO:0035324] (cellular component) References: PMID:9635420 Also known as: nurse cell ring canal, ovarian ring canal Definition: An intercellular bridge that connects the germline cells of a female cyst. Relationships: is a type of GO:0045172